{
  "gene_name": "Exosome complex component RRP45",
  "gene_symbol": "EXOSC9",
  "term_label": "TRAMP-dependent tRNA surveillance pathway",
  "term_id": "GO:0071038",
  "gene": "UniProtKB:Q06265"
}